{
  "gene_name": "Gamma-aminobutyric acid receptor subunit delta",
  "gene": "UniProtKB:O14764",
  "term_label": "chloride channel activity",
  "term_id": "GO:0005254",
  "gene_symbol": "GABRD"
}